positive regulation of thymocyte migration [GO:2000412] (biological process) Sources: GOC:mah Subtypes: positive regulation of fibronectin-dependent thymocyte migration [GO:2000415] Relationships: is a type of positive regulation of T cell migration [GO:2000406]; is a type of regulation of thymocyte migration [GO:2000410]; positively regulates GO:0072679 Also known as: positive regulation of thymic lymphocyte migration, positive regulation of immature T cell migration, positive regulation of immature T lymphocyte migration, positive regulation of immature T-cell migration, positive regulation of immature T-lymphocyte migration Definition: Any process that activates or increases the frequency, rate or extent of thymocyte migration.